{
  "gene_symbol": "OSBPL10",
  "term_id": "GO:0005829",
  "gene_name": "Oxysterol-binding protein-related protein 10",
  "gene": "UniProtKB:Q9BXB5",
  "term_label": "cytosol"
}